asymmetric neuroblast division [GO:0055059] (biological process) Definition: The process resulting in the physical partitioning and separation of a neuroblast into two daughter cells with different developmental potentials. Sources: GOC:dph Relationships: is a type of asymmetric cell division [GO:0008356]; is a type of cell fate commitment [GO:0045165]; is a type of neuroblast division [GO:0055057] Subtypes: GO:0055060